{
  "gene_name": "Phosphatidylinositol 4,5-bisphosphate 3-kinase catalytic subunit beta isoform",
  "gene_symbol": "PIK3CB",
  "gene": "UniProtKB:P42338",
  "term_id": "GO:0048015",
  "term_label": "phosphatidylinositol-mediated signaling"
}